{
  "gene_name": "Eukaryotic peptide chain release factor GTP-binding subunit ERF3A",
  "gene": "UniProtKB:P15170",
  "term_label": "GTPase activity",
  "term_id": "GO:0003924",
  "gene_symbol": "GSPT1"
}